{
  "term_id": "GO:0071880",
  "term_label": "adenylate cyclase-activating adrenergic receptor signaling pathway",
  "gene": "UniProtKB:P08588",
  "gene_name": "Beta-1 adrenergic receptor",
  "gene_symbol": "ADRB1"
}